regulation of eye pigmentation [GO:0048073] (biological process) Subtypes: negative regulation of eye pigmentation [GO:0048074], positive regulation of eye pigmentation [GO:0048075], regulation of compound eye pigmentation [GO:0048076] Sources: GOC:jid Definition: Any process that modulates the frequency, rate or extent of establishment of a pattern of pigment in the eye of an organism. Relationships: is a type of regulation of developmental pigmentation [GO:0048070]; regulates eye pigmentation [GO:0048069]